regulation of protein localization to ciliary membrane [GO:1903567] (biological process) Subtypes: negative regulation of protein localization to ciliary membrane [GO:1903568], positive regulation of protein localization to ciliary membrane [GO:1903569] Relationships: is a type of regulation of protein localization to cilium [GO:1903564]; is a type of regulation of protein localization to cell periphery [GO:1904375]; is a type of regulation of protein localization to membrane [GO:1905475]; regulates protein localization to ciliary membrane [GO:1903441] References: PMID:22072986 Sources: GOC:TermGenie, GOC:cilia, GOC:krc, GO_REF:0000058 Definition: Any process that modulates the frequency, rate or extent of protein localization to ciliary membrane. Also known as: regulation of protein localisation in ciliary membrane, regulation of protein localisation to ciliary membrane, regulation of protein localization in ciliary membrane